{
  "gene_symbol": "MAP10",
  "term_id": "GO:0097431",
  "term_label": "mitotic spindle pole",
  "gene": "UniProtKB:Q9P2G4",
  "gene_name": "Microtubule-associated protein 10"
}